{
  "gene_name": "Kinesin-like protein KIF25",
  "gene_symbol": "KIF25",
  "term_label": "microtubule binding",
  "gene": "UniProtKB:Q9UIL4",
  "term_id": "GO:0008017"
}